{
  "term_id": "GO:0004715",
  "term_label": "non-membrane spanning protein tyrosine kinase activity",
  "gene": "UniProtKB:P12931",
  "gene_symbol": "SRC",
  "gene_name": "Proto-oncogene tyrosine-protein kinase Src"
}